{
  "gene_symbol": "CXCL9",
  "term_label": "inflammatory response",
  "term_id": "GO:0006954",
  "gene": "UniProtKB:Q07325",
  "gene_name": "C-X-C motif chemokine 9"
}